{
  "gene_symbol": "IGHV3-15",
  "term_label": "Unknown cellular component",
  "gene_name": "Immunoglobulin heavy variable 3-15",
  "term_id": "UNKNOWN:0003",
  "gene": "UniProtKB:A0A0B4J1V0"
}